oxidoreductase activity, acting on hydrogen as donor, with a quinone or similar compound as acceptor [GO:0046994] (MF) Relationships: is a type of oxidoreductase activity, acting on hydrogen as donor [GO:0016695] Subtypes: hydrogen:quinone oxidoreductase activity [GO:0047067] Sources: GOC:jl Definition: Catalysis of an oxidation-reduction (redox) reaction in which hydrogen acts as an electron donor and reduces quinone or similar compound.